{
  "term_id": "UNKNOWN:0003",
  "gene": "UniProtKB:Q6AI08",
  "term_label": "Unknown cellular component",
  "gene_symbol": "HEATR6",
  "gene_name": "HEAT repeat-containing protein 6"
}